{
  "gene_symbol": "LRP4",
  "term_label": "plasma membrane",
  "term_id": "GO:0005886",
  "gene": "UniProtKB:O75096",
  "gene_name": "Low-density lipoprotein receptor-related protein 4"
}